glycine-tRNA ligase complex [GO:0009345] (cellular component) Relationships: is a type of GO:1902494; is part of cytoplasm [GO:0005737] References: PMID:15733854 Also known as: glycine-tRNA synthetase complex Definition: A multimeric enzyme complex which, in bacteria, is usually a tetramer of two alpha and two beta chains and in eukaryotes, is usually a homodimer. Functions in the ligation of glycine and tRNA(Gly) to form glycyl-tRNA(Gly).